{
  "term_id": "GO:0000139",
  "gene_name": "Calcium-transporting ATPase type 2C member 2",
  "term_label": "Golgi membrane",
  "gene": "UniProtKB:O75185",
  "gene_symbol": "ATP2C2"
}